tRNA C3-cytosine methylation [GO:0106217] (biological process) Relationships: is a type of tRNA methylation [GO:0030488] References: PMID:28655767 Definition: The process whereby a cytosine in a tRNA is methylated at position 3 of the cytosine.